regulation of catecholamine secretion [GO:0050433] (biological process) Relationships: is a type of regulation of amine transport [GO:0051952]; is a type of regulation of secretion by cell [GO:1903530]; regulates GO:0050432 Sources: GOC:ai Subtypes: regulation of dopamine secretion [GO:0014059], regulation of epinephrine secretion [GO:0014060], regulation of norepinephrine secretion [GO:0014061], negative regulation of catecholamine secretion [GO:0033604], positive regulation of catecholamine secretion [GO:0033605] Definition: Any process that modulates the frequency, rate or extent of the regulated release of catecholamines.